{
  "gene_symbol": "MARCHF4",
  "term_id": "GO:0005795",
  "gene_name": "E3 ubiquitin-protein ligase MARCHF4",
  "term_label": "Golgi stack",
  "gene": "UniProtKB:Q9P2E8"
}